virus tail, baseplate [GO:0098025] (cellular component) Definition: Multiprotein component at the distal (head) end of the virus tail to which fibers of tailed viruses may be attached. Note: Tail fibers are often attached to the baseplate of Caudovirales (tailed bacteriophages with dsDNA genomes). Sometimes referred to as the tail tip or tip structure in Siphoviridae. Also known as: bacteriophage baseplate, tail structure, tail tip Sources: GOC:bm, VZ:3957 Relationships: is a type of GO:0044423; is part of GO:0098015